{
  "gene_name": "ADP-ribosylation factor-related protein 1",
  "gene": "UniProtKB:Q13795",
  "term_label": "GTPase activity",
  "term_id": "GO:0003924",
  "gene_symbol": "ARFRP1"
}